{
  "term_label": "glutamyl-tRNA(Gln) amidotransferase complex",
  "gene": "UniProtKB:O75879",
  "term_id": "GO:0030956",
  "gene_symbol": "GATB",
  "gene_name": "Glutamyl-tRNA(Gln) amidotransferase subunit B, mitochondrial"
}